regulation of thyroid gland epithelial cell proliferation [GO:1904441] (biological process) Definition: Any process that modulates the frequency, rate or extent of thyroid gland epithelial cell proliferation. References: PMID:17646383 Sources: GOC:TermGenie, GO_REF:0000058 Also known as: regulation of Hurthle cell proliferation, regulation of thyroid follicular cell proliferation Relationships: is a type of regulation of epithelial cell proliferation [GO:0050678]; regulates thyroid gland epithelial cell proliferation [GO:1990789] Subtypes: negative regulation of thyroid gland epithelial cell proliferation [GO:1904442], positive regulation of thyroid gland epithelial cell proliferation [GO:1904443]